{
  "gene": "UniProtKB:Q13046",
  "gene_name": "Pregnancy-specific beta-1-glycoprotein 7",
  "term_id": "UNKNOWN:0002",
  "gene_symbol": "PSG7",
  "term_label": "Unknown biological process"
}